{
  "term_label": "axon terminus",
  "gene": "UniProtKB:O15130",
  "term_id": "GO:0043679",
  "gene_name": "Pro-FMRFamide-related neuropeptide FF",
  "gene_symbol": "NPFF"
}